{
  "gene_symbol": "JAK1",
  "term_label": "cytokine-mediated signaling pathway",
  "term_id": "GO:0019221",
  "gene_name": "Tyrosine-protein kinase JAK1",
  "gene": "UniProtKB:P23458"
}